DNA replication, removal of RNA primer [GO:0043137] (biological process) References: PMID:12424238 Sources: GOC:jl Definition: Removal of the Okazaki RNA primer from the lagging strand of replicating DNA, by a combination of the actions of DNA polymerase, DNA helicase and an endonuclease. Also known as: Okazaki initiator RNA removal Subtypes: removal of RNA primer involved in mitotic DNA replication [GO:1903469] Relationships: is a type of RNA catabolic process [GO:0006401]; is part of DNA replication [GO:0006260]